{
  "gene_name": "Secretoglobin family 1C member 1",
  "gene_symbol": "SCGB1C1",
  "gene": "UniProtKB:Q8TD33",
  "term_id": "UNKNOWN:0002",
  "term_label": "Unknown biological process"
}